{
  "gene": "UniProtKB:O60234",
  "term_id": "GO:0030864",
  "gene_symbol": "GMFG",
  "term_label": "cortical actin cytoskeleton",
  "gene_name": "Glia maturation factor gamma"
}